{
  "term_label": "DNA-binding transcription factor activity, RNA polymerase II-specific",
  "gene_name": "Zinc finger protein 587B",
  "term_id": "GO:0000981",
  "gene_symbol": "ZNF587B",
  "gene": "UniProtKB:E7ETH6"
}